{
  "term_id": "GO:0071782",
  "gene": "UniProtKB:Q8N5Y8",
  "gene_name": "Protein mono-ADP-ribosyltransferase PARP16",
  "term_label": "endoplasmic reticulum tubular network",
  "gene_symbol": "PARP16"
}